acyl-lipid (8-3)-desaturase activity [GO:0102866] (molecular function) Sources: EC:1.14.19.30 Also known as: Delta(5)-fatty-acid desaturase activity, acyl-lipid 5-desaturase activity, di-homo-gamma-linolenate delta5 desaturase activity Relationships: is_a GO:0016717 Definition: Catalysis of the reaction: an (8Z,11Z,14Z)-icosatrienoyl-containing glycerolipid + 2 Fe(II)-[cytochrome b5] + 2 H+ + O2 = (5Z,8Z,11Z,14Z)-eicosatetraenoyl-containing glycerolipid + 2 Fe(III)-[cytochrome b5] + 2 H2O. Also converts an (8Z,11Z,14Z,17Z)-eicosatetraenoyl-containing glycerolipid into a (5Z,8Z,11Z,14Z,17Z)-eicosapentaenoyl-containing glycerolipid.